{
  "term_label": "transcription regulator complex",
  "gene_symbol": "RCOR3",
  "term_id": "GO:0005667",
  "gene_name": "REST corepressor 3",
  "gene": "UniProtKB:Q9P2K3"
}